gap junction [GO:0005921] (cellular component) Definition: A cell-cell junction composed of pannexins or innexins and connexins, two different families of channel-forming proteins. Also known as: communicating junction, gap junction macula, gap junction plaque, macula communicans, zonula communicans, electrical synapse, electrotonic synapse, intercellular gap junction channel References: PMID:22366062 Sources: GOC:mah, GOC:mtg_muscle, ISBN:0815332181, Wikipedia:Gap_junction Relationships: is a type of cell-cell junction [GO:0005911]